{
  "term_id": "GO:0016020",
  "gene_name": "Taste receptor type 2 member 7",
  "gene_symbol": "TAS2R7",
  "gene": "UniProtKB:Q9NYW3",
  "term_label": "membrane"
}